mannitol-1-phosphate 5-dehydrogenase activity [GO:0008926] (molecular function) Definition: Catalysis of the reaction: D-mannitol 1-phosphate + NAD+ = D-fructose 6-phosphate + NADH + H+. Note: Note that this term has a MetaCyc pathway reference as the pathway only has a single step. Sources: EC:1.1.1.17 Relationships: is a type of oxidoreductase activity, acting on the CH-OH group of donors, NAD or NADP as acceptor [GO:0016616]